negative regulation of macrophage activation [GO:0043031] (biological process) Relationships: is a type of negative regulation of leukocyte activation [GO:0002695]; is_a regulation of macrophage activation [GO:0043030]; negatively regulates macrophage activation [GO:0042116] Sources: GOC:jl Subtypes: GO:1903979 Also known as: down regulation of macrophage activation, down-regulation of macrophage activation, downregulation of macrophage activation, negative regulation of macrophage polarization, inhibition of macrophage activation Definition: Any process that stops, prevents, or reduces the frequency, rate or extent of macrophage activation.